{
  "gene": "UniProtKB:P46100",
  "term_id": "GO:0031297",
  "gene_name": "Transcriptional regulator ATRX",
  "gene_symbol": "ATRX",
  "term_label": "replication fork processing"
}